{
  "gene_name": "Double homeobox protein 4-like protein 4",
  "term_id": "GO:0000981",
  "gene": "UniProtKB:P0CJ87",
  "term_label": "DNA-binding transcription factor activity, RNA polymerase II-specific",
  "gene_symbol": "DUX4L4"
}